{
  "gene_symbol": "RHOBTB1",
  "term_label": "cell projection",
  "term_id": "GO:0042995",
  "gene": "UniProtKB:O94844",
  "gene_name": "Rho-related BTB domain-containing protein 1"
}